syncytium formation [GO:0006949] (BP) Subtypes: GO:0000768, syncytium formation by mitosis without cytokinesis [GO:0000769] Sources: ISBN:0198506732 Definition: The formation of a syncytium, a mass of cytoplasm containing several nuclei enclosed within a single plasma membrane. Syncytia are normally derived from single cells that fuse or fail to complete cell division. Relationships: is_a cellular process [GO:0009987]; is a type of GO:0048646